cytoplasmic side of trans-Golgi network transport vesicle membrane [GO:0098541] (cellular component) Definition: The side (leaflet) of the trans-Golgi network transport vesicle membrane that faces the cytoplasm. Sources: GOC:ab Relationships: is a type of cytoplasmic side of transport vesicle membrane [GO:0098539]; is part of GO:0012510 Also known as: external side of trans-Golgi network transport vesicle membrane